{
  "gene_name": "Chloride anion exchanger",
  "gene": "UniProtKB:P40879",
  "term_id": "GO:1902358",
  "gene_symbol": "SLC26A3",
  "term_label": "sulfate transmembrane transport"
}